RNA repair [GO:0042245] (biological process) References: PMID:11000254, PMID:11070075 Sources: UniProtKB-KW:KW-0692 Relationships: is_a RNA metabolic process [GO:0016070] Definition: Any process that results in the repair of damaged RNA.